{
  "term_id": "UNKNOWN:0001",
  "term_label": "Unknown molecular function",
  "gene_name": "Uncharacterized protein C10orf82",
  "gene_symbol": "C10orf82",
  "gene": "UniProtKB:Q8WW14"
}